{
  "gene": "UniProtKB:Q5JUQ0",
  "gene_name": "Protein FAM78A",
  "term_label": "Unknown molecular function",
  "gene_symbol": "FAM78A",
  "term_id": "UNKNOWN:0001"
}